regulation of sinapate ester biosynthetic process [GO:1903085] (biological process) Subtypes: negative regulation of sinapate ester biosynthetic process [GO:1903086] Definition: Any process that modulates the frequency, rate or extent of sinapate ester biosynthesis. References: PMID:11080161 Sources: GOC:TermGenie, GO_REF:0000058 Relationships: is a type of GO:1900376; is a type of regulation of phenylpropanoid metabolic process [GO:2000762]; regulates sinapate ester biosynthetic process [GO:0033525] Also known as: regulation of sinapate ester anabolism, regulation of sinapate ester biosynthesis, regulation of sinapate ester formation, regulation of sinapate ester synthesis